{
  "term_id": "UNKNOWN:0002",
  "gene_name": "Zinc finger imprinted 2",
  "gene": "UniProtKB:Q9NZV7",
  "term_label": "Unknown biological process",
  "gene_symbol": "ZIM2"
}